{
  "gene_symbol": "NCBP3",
  "gene": "UniProtKB:Q53F19",
  "term_label": "Unknown biological process",
  "term_id": "UNKNOWN:0002",
  "gene_name": "Nuclear cap-binding protein subunit 3"
}